{
  "term_label": "alpha-tubulin binding",
  "gene_name": "Trafficking protein particle complex subunit 14",
  "term_id": "GO:0043014",
  "gene_symbol": "TRAPPC14",
  "gene": "UniProtKB:Q8WVR3"
}